{
  "gene": "UniProtKB:P0DUX0",
  "term_label": "Unknown cellular component",
  "gene_symbol": "SPDYE10",
  "term_id": "UNKNOWN:0003",
  "gene_name": "Speedy protein E10"
}